posterior lateral line development [GO:0048916] (biological process) Definition: The process whose specific outcome is the progression of the posterior lateral line over time, from its formation to the mature structure. The posterior lateral line consists of small sensory patches (neuromasts) located superficially on the skin or just under the skin in fluid-filled canals on the body and trunk of all fishes and most amphibians. The posterior lateral line develops from cranial ectodermal placodes situated behind the ear. Sources: ISBN:0125296509 Also known as: PLL development Relationships: is_a lateral line development [GO:0048882]; is part of posterior lateral line system development [GO:0048915]